{
  "gene_name": "Surfactant-associated protein 3",
  "gene_symbol": "SFTA3",
  "term_id": "GO:0005615",
  "term_label": "extracellular space",
  "gene": "UniProtKB:P0C7M3"
}